neuron-neuron synaptic transmission [GO:0007270] (biological process) Relationships: is a type of chemical synaptic transmission [GO:0007268] Also known as: nerve-nerve synaptic transmission Definition: The process of synaptic transmission from a neuron to another neuron across a synapse. Sources: GOC:add, GOC:dos, GOC:jl, MeSH:D009435